{
  "term_id": "GO:0005737",
  "gene_symbol": "ACOT7",
  "term_label": "cytoplasm",
  "gene": "UniProtKB:O00154",
  "gene_name": "Cytosolic acyl coenzyme A thioester hydrolase"
}